{
  "gene": "UniProtKB:P15153",
  "gene_name": "Ras-related C3 botulinum toxin substrate 2",
  "term_id": "GO:0031410",
  "gene_symbol": "RAC2",
  "term_label": "cytoplasmic vesicle"
}